epiboly involved in gastrulation with mouth forming second [GO:0055113] (biological process) Sources: ISBN:0878932437 Regulation: RO_0002211 by regulation of epiboly involved in gastrulation with mouth forming second [GO:1904086]; negatively regulated by negative regulation of epiboly involved in gastrulation with mouth forming second [GO:1904087]; positively regulated by GO:1904088 Relationships: is a type of embryonic morphogenesis [GO:0048598]; is a type of GO:0090504; is part of GO:0001702 Definition: The expansion of one cell sheet over other cells involved in deuterostomic gastrulation.